response to quercetin [GO:1905235] (biological process) Relationships: is a type of GO:1905395 References: PMID:24914722 Sources: GOC:TermGenie, GO_REF:0000071 Subtypes: cellular response to quercetin [GO:1905236] Definition: Any process that results in a change in state or activity of a cell or an organism (in terms of movement, secretion, enzyme production, gene expression, etc.) as a result of a quercetin stimulus.